{
  "gene": "UniProtKB:O14495",
  "gene_name": "Phospholipid phosphatase 3",
  "gene_symbol": "PLPP3",
  "term_label": "signal transduction",
  "term_id": "GO:0007165"
}